{
  "gene_symbol": "NDC1",
  "gene": "UniProtKB:Q9BTX1",
  "term_label": "protein-macromolecule adaptor activity",
  "term_id": "GO:0030674",
  "gene_name": "Nucleoporin NDC1"
}